positive regulation of mannotriose transport [GO:1900329] (biological process) Sources: GOC:TermGenie, GOC:mengo_curators Relationships: is a type of positive regulation of transport [GO:0051050]; is a type of regulation of mannotriose transport [GO:1900327]; positively regulates mannotriose transport [GO:2001095] Definition: Any process that activates or increases the frequency, rate or extent of mannotriose transport. Also known as: up regulation of mannotriose transport, up-regulation of mannotriose transport, upregulation of mannotriose transport, activation of mannotriose transport